{
  "term_id": "GO:0005219",
  "gene_symbol": "RYR1",
  "gene": "UniProtKB:P21817",
  "gene_name": "Ryanodine receptor 1",
  "term_label": "ryanodine-sensitive calcium-release channel activity"
}